{
  "term_id": "GO:0034362",
  "gene": "UniProtKB:O95445",
  "gene_symbol": "APOM",
  "gene_name": "Apolipoprotein M",
  "term_label": "low-density lipoprotein particle"
}